{
  "gene": "UniProtKB:Q9HCP6",
  "term_label": "regulation of protein modification process",
  "term_id": "GO:0031399",
  "gene_name": "Protein-cysteine N-palmitoyltransferase HHAT-like protein",
  "gene_symbol": "HHATL"
}